{
  "term_label": "Unknown biological process",
  "gene": "UniProtKB:Q8TDM0",
  "gene_symbol": "BCAS4",
  "term_id": "UNKNOWN:0002",
  "gene_name": "Breast carcinoma-amplified sequence 4"
}